oxidized DNA binding [GO:0032356] (molecular function) Definition: Binding to a DNA region containing an oxidized residue. Sources: GOC:vk Also known as: oxidised DNA binding Relationships: is a type of damaged DNA binding [GO:0003684] Subtypes: oxidized purine DNA binding [GO:0032357], oxidized pyrimidine DNA binding [GO:0032358]